basal distal dendrite [GO:0150016] (CC) References: PMID:17046728, PMID:1720142, PMID:20629984, PMID:22683681, PMID:9214543 Sources: GOC:aruk, GOC:bc Relationships: is a type of basal dendrite [GO:0097441]; is a type of distal dendrite [GO:0150002] Definition: Any dendrite in a dendritic tree that emerges near the basal pole of a neuron (e.g. in bipolar neurons, basal dendrites are either on the same side of the soma as the axon, or project toward the axon), and which is farthest away from the neuronal cell body (the soma).